{
  "term_label": "potassium channel regulator activity",
  "gene_symbol": "KCNE5",
  "gene": "UniProtKB:Q9UJ90",
  "gene_name": "Potassium voltage-gated channel subfamily E regulatory beta subunit 5",
  "term_id": "GO:0015459"
}